{
  "term_id": "GO:0007411",
  "term_label": "axon guidance",
  "gene_name": "Ephrin-A3",
  "gene": "UniProtKB:P52797",
  "gene_symbol": "EFNA3"
}